central tolerance induction to nonself antigen [GO:0002463] (biological process) Relationships: is a type of tolerance induction to nonself antigen [GO:0002462]; is a type of central tolerance induction [GO:0002508] References: PMID:12547504 Sources: GOC:jal Definition: Tolerance induction to nonself antigens in the central lymphoid organs.